{
  "gene_name": "Keratin-associated protein 4-1",
  "gene": "UniProtKB:Q9BYQ7",
  "term_label": "Unknown biological process",
  "gene_symbol": "KRTAP4-1",
  "term_id": "UNKNOWN:0002"
}